ABC-type putrescine transporter activity [GO:0015594] (MF) Definition: Catalysis of the reaction: putrescine(out) + ATP + H2O = putrescine(in) + ADP + phosphate + H+. Sources: RHEA:29995 Also known as: putrescine porter activity, putrescine-importing ATPase activity, ATPase-coupled putrescine transmembrane transporter activity Relationships: is a type of ABC-type polyamine transporter activity [GO:0015417]; is_a putrescine transmembrane transporter activity [GO:0015489]